{
  "term_label": "maturation of LSU-rRNA from tricistronic rRNA transcript (SSU-rRNA, 5.8S rRNA, LSU-rRNA)",
  "gene_name": "Zinc finger HIT domain-containing protein 3",
  "term_id": "GO:0000463",
  "gene_symbol": "ZNHIT3",
  "gene": "UniProtKB:Q15649"
}